{
  "gene_name": "Protein shortage in chiasmata 1 ortholog",
  "gene": "UniProtKB:Q5VXU9",
  "gene_symbol": "SHOC1",
  "term_id": "GO:0000794",
  "term_label": "condensed nuclear chromosome"
}